{
  "gene": "UniProtKB:Q5JTC6",
  "term_id": "GO:0008013",
  "gene_symbol": "AMER1",
  "term_label": "beta-catenin binding",
  "gene_name": "APC membrane recruitment protein 1"
}